positive regulation of iridophore differentiation [GO:0050945] (biological process) Relationships: is a type of regulation of iridophore differentiation [GO:0050937]; is a type of positive regulation of pigment cell differentiation [GO:0050942]; positively regulates iridophore differentiation [GO:0050935] Definition: Any process that activates or increases the frequency, rate or extent of iridophore differentiation. Sources: GOC:ai Also known as: up regulation of iridophore differentiation, up-regulation of iridophore differentiation, upregulation of iridophore differentiation, activation of iridophore differentiation, stimulation of iridophore differentiation